{
  "gene_symbol": "IGLV3-1",
  "gene": "UniProtKB:P01715",
  "term_id": "GO:0006955",
  "term_label": "immune response",
  "gene_name": "Immunoglobulin lambda variable 3-1"
}